{
  "term_label": "Unknown molecular function",
  "gene": "UniProtKB:Q96EL2",
  "gene_symbol": "MRPS24",
  "gene_name": "Small ribosomal subunit protein uS3m",
  "term_id": "UNKNOWN:0001"
}